lateral sprouting from an epithelium [GO:0060601] (biological process) Relationships: is a type of morphogenesis of an epithelium [GO:0002009]; is part of morphogenesis of a branching epithelium [GO:0061138] Sources: GOC:dph Subtypes: lateral sprouting involved in lung morphogenesis [GO:0060490], prostatic bud formation [GO:0060513], lateral sprouting involved in mammary gland duct morphogenesis [GO:0060599], lateral sprouting involved in ureteric bud morphogenesis [GO:0060680] Definition: The process in which a branch forms along the side of an epithelium.